viral capsid assembly [GO:0019069] (biological process) References: PMID:22615368 Sources: ISBN:0781702534 Relationships: is a type of viral process [GO:0016032]; is part of virion assembly [GO:0019068] Subtypes: nuclear capsid assembly [GO:0039708], cytoplasmic capsid assembly [GO:0039709] Definition: The assembly of a virus capsid from its protein subunits.